{
  "term_label": "Unknown molecular function",
  "gene": "UniProtKB:Q09MP3",
  "term_id": "UNKNOWN:0001",
  "gene_symbol": "RAD51AP2",
  "gene_name": "RAD51-associated protein 2"
}